{
  "term_label": "cortical actin cytoskeleton",
  "term_id": "GO:0030864",
  "gene_symbol": "SPTBN4",
  "gene": "UniProtKB:Q9H254",
  "gene_name": "Spectrin beta chain, non-erythrocytic 4"
}